interleukin-7 receptor activity [GO:0004917] (molecular function) Also known as: IL-7 receptor activity, IL-7R Definition: Combining with interleukin-7 and transmitting the signal from one side of the membrane to the other to initiate a change in cell activity. Relationships: is a type of GO:0004896; is part of GO:0038111; BFO_0000051 interleukin-7 binding [GO:0019982] Sources: GOC:jl, GOC:signaling